{
  "gene_symbol": "DNAL4",
  "term_id": "UNKNOWN:0002",
  "gene_name": "Dynein axonemal light chain 4",
  "term_label": "Unknown biological process",
  "gene": "UniProtKB:O96015"
}